galanin receptor activity [GO:0004966] (molecular function) Sources: GOC:ai Relationships: is a type of neuropeptide receptor activity [GO:0008188] Definition: Combining with galanin to initiate a change in cell activity.